{
  "gene_symbol": "MTDH",
  "term_id": "GO:0051059",
  "term_label": "NF-kappaB binding",
  "gene": "UniProtKB:Q86UE4",
  "gene_name": "Protein LYRIC"
}